{
  "term_id": "GO:0006413",
  "gene": "UniProtKB:P55884",
  "gene_name": "Eukaryotic translation initiation factor 3 subunit B",
  "term_label": "translational initiation",
  "gene_symbol": "EIF3B"
}